{
  "gene_symbol": "ZNF479",
  "gene_name": "Zinc finger protein 479",
  "gene": "UniProtKB:Q96JC4",
  "term_label": "DNA-binding transcription factor activity, RNA polymerase II-specific",
  "term_id": "GO:0000981"
}